{
  "gene": "UniProtKB:Q9UGC7",
  "gene_name": "Peptide chain release factor 1-like, mitochondrial",
  "term_label": "mitochondrial translational termination",
  "gene_symbol": "MTRF1L",
  "term_id": "GO:0070126"
}